{
  "gene_name": "Chitinase-3-like protein 1",
  "term_id": "GO:0005576",
  "gene_symbol": "CHI3L1",
  "gene": "UniProtKB:P36222",
  "term_label": "extracellular region"
}